{
  "gene_name": "Equilibrative nucleoside transporter 2",
  "term_label": "hypoxanthine transport",
  "gene": "UniProtKB:Q14542",
  "gene_symbol": "SLC29A2",
  "term_id": "GO:0035344"
}